{
  "term_label": "exocyst",
  "gene_symbol": "EXOC2",
  "term_id": "GO:0000145",
  "gene_name": "Exocyst complex component 2",
  "gene": "UniProtKB:Q96KP1"
}